{
  "gene": "UniProtKB:Q15398",
  "gene_name": "Disks large-associated protein 5",
  "term_label": "nucleus",
  "gene_symbol": "DLGAP5",
  "term_id": "GO:0005634"
}